hepatocyte differentiation [GO:0070365] (biological process) Also known as: liver cell differentiation Relationships: is a type of GO:0030855; is part of GO:0001889 Regulation: regulated by GO:0070366; negatively regulated by negative regulation of hepatocyte differentiation [GO:0070367]; positively regulated by positive regulation of hepatocyte differentiation [GO:0070368] Definition: The process in which a relatively unspecialized cell acquires the specialized features of a hepatocyte. A hepatocyte is specialized epithelial cell that is organized into interconnected plates called lobules, and is the main structural component of the liver. References: PMID:7588884 Sources: CL:0000182